{
  "term_id": "GO:0000978",
  "term_label": "RNA polymerase II cis-regulatory region sequence-specific DNA binding",
  "gene_symbol": "HIC2",
  "gene": "UniProtKB:Q96JB3",
  "gene_name": "Hypermethylated in cancer 2 protein"
}